{
  "gene_symbol": "CLASP2",
  "term_label": "spindle microtubule",
  "gene": "UniProtKB:O75122",
  "gene_name": "CLIP-associating protein 2",
  "term_id": "GO:0005876"
}